{
  "term_id": "GO:0005667",
  "term_label": "transcription regulator complex",
  "gene_symbol": "PROP1",
  "gene": "UniProtKB:O75360",
  "gene_name": "Homeobox protein prophet of Pit-1"
}